{
  "gene_name": "Zinc finger and BTB domain-containing protein 47",
  "term_id": "GO:0005634",
  "gene_symbol": "ZBTB47",
  "term_label": "nucleus",
  "gene": "UniProtKB:Q9UFB7"
}